amino acid transport complex [GO:1990184] (cellular component) Relationships: is a type of GO:0098797 References: PMID:14668347 Sources: GOC:kmv Definition: A heteromeric protein complex consisting of a multi-transmembrane spanning subunit (the light chain) and a type II glycoprotein subunit (the heavy chain) that functions to transport amino acids across a plasma membrane.